{
  "gene": "UniProtKB:Q5TCX8",
  "term_id": "GO:0005737",
  "term_label": "cytoplasm",
  "gene_symbol": "MAP3K21",
  "gene_name": "Mitogen-activated protein kinase kinase kinase 21"
}